{
  "term_label": "cytoplasm",
  "gene_name": "Ankyrin repeat and IBR domain-containing protein 1",
  "term_id": "GO:0005737",
  "gene_symbol": "ANKIB1",
  "gene": "UniProtKB:Q9P2G1"
}